{
  "gene": "UniProtKB:Q96KC9",
  "gene_name": "Calcium-binding and spermatid-specific protein 1",
  "term_label": "spermatogenesis",
  "term_id": "GO:0007283",
  "gene_symbol": "CABS1"
}